interphase [GO:0051325] (biological process) Definition: The cell cycle phase following cytokinesis which begins with G1 phase, proceeds through S phase and G2 phase and ends when prophase of meiosis or mitosis begins. During interphase the cell readies itself for meiosis or mitosis and the replication of its DNA occurs. Sources: GOC:mtg_cell_cycle Subtypes: meiotic interphase [GO:0051328], mitotic interphase [GO:0051329] Note: Note that this term should not be used for direct annotation. If you are trying to make an annotation to x phase, it is likely that the correct annotation is 'regulation of x/y phase transition' or to a process which occurs during the reported phase (i.e mitotic DNA replication for mitotic S-phase). To capture the phase when a specific location or process is observed, the phase term can be used in an annotation extension (PMID:24885854) applied to a cellular component term (with the relation exists_during) or a biological process term (with the relation happens_during). Relationships: is a type of cell cycle phase [GO:0022403] Also known as: resting phase, karyostasis